{
  "term_id": "GO:0005730",
  "term_label": "nucleolus",
  "gene_symbol": "RPF1",
  "gene": "UniProtKB:Q9H9Y2",
  "gene_name": "Ribosome production factor 1"
}